tRNA wobble position uridine thiolation [GO:0002143] (biological process) Relationships: is a type of tRNA wobble uridine modification [GO:0002098]; is a type of GO:0034227 References: PMID:16871210 Note: In E. coli, the first step of the reaction is reductive elimination of sulfur from L-cysteine by IscS cysteine desulfurase to form an enzyme-bound cysteine-persulfide intermediate. Then, five essential gene products, TusA, TusB, TusC, TusD and TusE, mediate a sulfur relay that delivers the terminal sulfur of persulfide from IscS to MnmA12. The last protein, MnmA catalyzes the transfer of the sulfur from IscS to an ATP activated U34 of the tRNA. Also known as: tRNA wobble uridine thiolation, wobble position s2U biosynthesis Subtypes: mitochondrial tRNA wobble position uridine thiolation [GO:1990799] Definition: The process in which a uridine residue at position 34 in the anticodon of a tRNA is post-transcriptionally thiolated at the C2 position. This process involves transfer of a sulfur from cysteine to position C2 by several steps.